mRNA trans splicing, SL addition [GO:0045291] (biological process) Definition: The joining together of two independently transcribed RNAs, where the one that provides the 5' portion of the final mRNA is from a splice leader RNA (SL-RNA). The SL-RNA, or mini-exon donor sequence, is added to the 5'-end of the acceptor RNA molecule which provides the mRNA body. Relationships: is a type of mRNA trans splicing, via spliceosome [GO:0000365] Also known as: nuclear mRNA trans splicing, SL addition, nuclear mRNA trans splicing, spliced leader addition References: PMID:2675423 Sources: GOC:krc, ISBN:0879695897